histone methyltransferase inhibitor activity [GO:0180000] (molecular function) Definition: Binds to and stops, prevents or reduces the activity of a histone methyltransferase. References: PMID:30923826 Relationships: is a type of GO:0004857